{
  "gene_symbol": "SELENOT",
  "gene_name": "Thioredoxin reductase-like selenoprotein T",
  "term_label": "thioredoxin-disulfide reductase (NADPH) activity",
  "term_id": "GO:0004791",
  "gene": "UniProtKB:P62341"
}